{
  "term_label": "SNAP receptor activity",
  "gene_symbol": "VAMP7",
  "gene_name": "Vesicle-associated membrane protein 7",
  "gene": "UniProtKB:P51809",
  "term_id": "GO:0005484"
}